pancreatic stellate cell proliferation [GO:0072343] (biological process) References: PMID:17200706 Sources: CL:0002410, GOC:mah Definition: The multiplication or reproduction of pancreatic stellate cells, resulting in the expansion of a pancreatic stellate cell population. Pancreatic stellate cells are found in the periacinar space of the exocrine pancreas and in perivascular and periductal regions of the pancreas, and have long cytoplasmic processes that encircle the base of the acinus. Regulation: regulated by GO:2000229; negatively regulated by negative regulation of pancreatic stellate cell proliferation [GO:2000230]; positively regulated by GO:2000231 Relationships: is a type of fibroblast proliferation [GO:0048144]